{
  "gene": "UniProtKB:Q9UKF5",
  "term_id": "GO:0004222",
  "gene_name": "Disintegrin and metalloproteinase domain-containing protein 29",
  "gene_symbol": "ADAM29",
  "term_label": "metalloendopeptidase activity"
}